fructosyl-amino acid oxidase activity [GO:0051700] (molecular function) Relationships: is a type of oxidoreductase activity, acting on the CH-NH group of donors, oxygen as acceptor [GO:0016647] References: PMID:16233628 Also known as: FAOD activity Definition: Catalysis of the reaction: fructosyl-amino acid + O2 = corresponding amino acid + glucosone + H2O2.